copper ion binding [GO:0005507] (MF) Subtypes: cupric ion binding [GO:1903135], cuprous ion binding [GO:1903136] Definition: Binding to a copper (Cu) ion. Relationships: is a type of transition metal ion binding [GO:0046914] Sources: GOC:ai Also known as: copper/cadmium binding, copper binding